{
  "gene_name": "Forkhead box protein I3",
  "term_label": "RNA polymerase II cis-regulatory region sequence-specific DNA binding",
  "term_id": "GO:0000978",
  "gene": "UniProtKB:A8MTJ6",
  "gene_symbol": "FOXI3"
}